{
  "gene": "UniProtKB:Q99741",
  "term_label": "mitotic DNA replication checkpoint signaling",
  "term_id": "GO:0033314",
  "gene_name": "Cell division control protein 6 homolog",
  "gene_symbol": "CDC6"
}